retrograde trans-synaptic signaling by neuropeptide, modulating synaptic transmission [GO:0099083] (biological process) Definition: Modulation of synaptic transmission by cell-cell signaling across the synaptic cleft from postsynapse to presynapse, mediated by a neuropeptide. References: PMID:19448629 Sources: GOC:PARL, GOC:bf, GOC:dos Note: Note that this term was created for the SynGO project, and will be obsoleted when the SynGO annotations are made in Noctua. Relationships: is a type of retrograde trans-synaptic signaling by neuropeptide [GO:0099082]; is a type of trans-synaptic signaling by neuropeptide, modulating synaptic transmission [GO:0099551]